{
  "gene": "UniProtKB:Q9Y3F4",
  "term_id": "GO:0003723",
  "gene_name": "Serine-threonine kinase receptor-associated protein",
  "gene_symbol": "STRAP",
  "term_label": "RNA binding"
}